{
  "gene_name": "Zinc finger protein 684",
  "term_id": "GO:0000977",
  "gene": "UniProtKB:Q5T5D7",
  "gene_symbol": "ZNF684",
  "term_label": "RNA polymerase II transcription regulatory region sequence-specific DNA binding"
}